{
  "gene_symbol": "MRPS9",
  "gene": "UniProtKB:P82933",
  "term_label": "Unknown biological process",
  "gene_name": "Small ribosomal subunit protein uS9m",
  "term_id": "UNKNOWN:0002"
}